{
  "gene_name": "Transcription factor 7-like 2",
  "term_label": "catenin-TCF7L2 complex",
  "gene": "UniProtKB:Q9NQB0",
  "gene_symbol": "TCF7L2",
  "term_id": "GO:0071664"
}